{
  "gene_name": "ZW10 interactor",
  "gene": "UniProtKB:O95229",
  "term_label": "establishment of localization in cell",
  "gene_symbol": "ZWINT",
  "term_id": "GO:0051649"
}